{
  "term_label": "DNA-binding transcription factor activity, RNA polymerase II-specific",
  "gene_name": "Iroquois-class homeodomain protein IRX-6",
  "gene": "UniProtKB:P78412",
  "gene_symbol": "IRX6",
  "term_id": "GO:0000981"
}